{
  "gene": "UniProtKB:Q9HCP0",
  "term_label": "positive regulation of canonical Wnt signaling pathway",
  "term_id": "GO:0090263",
  "gene_symbol": "CSNK1G1",
  "gene_name": "Casein kinase I isoform gamma-1"
}